{
  "gene_symbol": "IDE",
  "term_id": "GO:0004222",
  "gene": "UniProtKB:P14735",
  "term_label": "metalloendopeptidase activity",
  "gene_name": "Insulin-degrading enzyme"
}